{
  "term_id": "GO:0005739",
  "gene_name": "NADH-cytochrome b5 reductase 1",
  "term_label": "mitochondrion",
  "gene_symbol": "CYB5R1",
  "gene": "UniProtKB:Q9UHQ9"
}